{
  "gene": "UniProtKB:Q13641",
  "gene_name": "Trophoblast glycoprotein",
  "term_label": "plasma membrane",
  "gene_symbol": "TPBG",
  "term_id": "GO:0005886"
}